RNAi effector complex [GO:0031332] (cellular component) References: PMID:14704433 Sources: GOC:mah Subtypes: RISC complex [GO:0016442], RITS complex [GO:0030958], ARC complex [GO:0033167] Relationships: is a type of GO:1990904 Definition: Any protein complex that mediates the effects of small interfering RNAs on gene expression. Most known examples contain one or more members of the Argonaute family of proteins.